{
  "gene_symbol": "OR10H4",
  "term_label": "plasma membrane",
  "term_id": "GO:0005886",
  "gene": "UniProtKB:Q8NGA5",
  "gene_name": "Olfactory receptor 10H4"
}